ethylene biosynthetic process [GO:0009693] (BP) Definition: The chemical reactions and pathways resulting in the formation of ethylene (C2-H4, ethene), a simple hydrocarbon gas that can function in plants as a growth regulator. Sources: ISBN:0387969845 Also known as: ethene biosynthesis, ethene biosynthesis from L-methionine, ethene biosynthetic process, ethene biosynthetic process from L-methionine, ethylene anabolism, ethylene biosynthesis, ethylene biosynthesis from L-methionine, ethylene biosynthetic process from L-methionine, ethylene formation, ethylene synthesis Relationships: is a type of ethylene metabolic process [GO:0009692]; is a type of alkene biosynthetic process [GO:0043450] Subtypes: GO:0043272 Regulation: regulated by regulation of ethylene biosynthetic process [GO:0010364]; positively regulated by positive regulation of ethylene biosynthetic process [GO:0010365]; negatively regulated by GO:0010366